{
  "gene": "UniProtKB:P35354",
  "term_id": "GO:0043005",
  "gene_symbol": "PTGS2",
  "term_label": "neuron projection",
  "gene_name": "Prostaglandin G_H synthase 2"
}